{
  "term_label": "centriole",
  "gene_name": "Serologically defined colon cancer antigen 8",
  "gene": "UniProtKB:Q86SQ7",
  "gene_symbol": "SDCCAG8",
  "term_id": "GO:0005814"
}